cyst wall [GO:0097570] (cellular component) References: PMID:15134259, PMID:2026212 Sources: GOC:giardia, Wikipedia:Microbial_cyst Definition: The specialized envelope lying outside the cell membrane of a cyst. A cyst is a resting or dormant stage of a microorganism, usually a bacterium or a protist or rarely an invertebrate animal, that helps the organism to survive in unfavorable environmental conditions. In protists such as protozoan parasites alternating cystic- and non-cystic stages, the cyst wall is usually composed of carbohydrates and proteins. Relationships: is a type of GO:0005618